{
  "gene_symbol": "POMP",
  "term_id": "GO:0005634",
  "gene": "UniProtKB:Q9Y244",
  "term_label": "nucleus",
  "gene_name": "Proteasome maturation protein"
}